{
  "gene_name": "Cytochrome c",
  "gene_symbol": "CYCS",
  "term_label": "electron transfer activity",
  "gene": "UniProtKB:P99999",
  "term_id": "GO:0009055"
}